{
  "gene": "UniProtKB:P51809",
  "gene_name": "Vesicle-associated membrane protein 7",
  "term_label": "SNARE complex",
  "term_id": "GO:0031201",
  "gene_symbol": "VAMP7"
}